{
  "gene_name": "Cystatin-SN",
  "term_id": "GO:0005737",
  "gene_symbol": "CST1",
  "term_label": "cytoplasm",
  "gene": "UniProtKB:P01037"
}